{
  "gene_name": "[Pyruvate dehydrogenase (acetyl-transferring)] kinase isozyme 3, mitochondrial",
  "gene_symbol": "PDK3",
  "term_label": "pyruvate dehydrogenase (acetyl-transferring) kinase activity",
  "gene": "UniProtKB:Q15120",
  "term_id": "GO:0004740"
}